{
  "term_label": "regulation of transcription by RNA polymerase II",
  "gene_name": "Nuclear body protein SP140",
  "gene": "UniProtKB:Q13342",
  "term_id": "GO:0006357",
  "gene_symbol": "SP140"
}